protein transmembrane transporter activity [GO:0008320] (molecular function) Definition: Enables the transfer of a protein from one side of a membrane to the other. Sources: GOC:jl Also known as: protein channel activity Relationships: is a type of macromolecule transmembrane transporter activity [GO:0022884]; is a type of GO:0140318; is part of protein transmembrane transport [GO:0071806] Subtypes: GO:0009977, protein-transporting ATPase activity [GO:0015450], lactoferrin transmembrane transporter activity [GO:0033569]